ABC-type ferric iron transporter activity [GO:0015408] (molecular function) Sources: RHEA:12332 Also known as: ABC-type Fe3+ transporter, ferric ABC transporter, ATPase-coupled ferric iron transmembrane transporter activity, Fe3+-transporting ATPase activity, ferric transporting ATPase activity, ferric-transporting ATPase activity Relationships: is_a ferric iron transmembrane transporter activity [GO:0015091]; is a type of ATPase-coupled monoatomic cation transmembrane transporter activity [GO:0019829]; is a type of GO:0140359 Definition: Enables the transfer of a solute or solutes from one side of a membrane to the other according to the reaction: ATP + H2O + Fe3+(out) = ADP + phosphate + Fe3+(in).